{
  "term_id": "UNKNOWN:0003",
  "gene": "UniProtKB:Q92530",
  "gene_symbol": "PSMF1",
  "gene_name": "Proteasome inhibitor PI31 subunit",
  "term_label": "Unknown cellular component"
}